{
  "gene_symbol": "TMEM165",
  "gene_name": "Transmembrane protein 165",
  "gene": "UniProtKB:Q9HC07",
  "term_label": "calcium ion transmembrane transport",
  "term_id": "GO:0070588"
}